{
  "gene_symbol": "ARMC6",
  "gene_name": "Armadillo repeat-containing protein 6",
  "term_label": "Unknown cellular component",
  "term_id": "UNKNOWN:0003",
  "gene": "UniProtKB:Q6NXE6"
}